purine deoxyribonucleoside triphosphate metabolic process [GO:0009215] (biological process) Definition: The chemical reactions and pathways involving purine deoxyribonucleoside triphosphate, a compound consisting of a purine base linked to a deoxyribose sugar esterified with triphosphate on the sugar. Sources: GOC:go_curators, ISBN:0198506732 Also known as: purine deoxyribonucleoside triphosphate metabolism Relationships: is a type of purine nucleoside triphosphate metabolic process [GO:0009144]; is a type of deoxyribonucleoside triphosphate metabolic process [GO:0009200] Subtypes: GO:0009216, purine deoxyribonucleoside triphosphate catabolic process [GO:0009217], GO:0046060, dGTP metabolic process [GO:0046070]